{
  "term_id": "GO:0045087",
  "gene_name": "Protein WFDC10B",
  "term_label": "innate immune response",
  "gene": "UniProtKB:Q8IUB3",
  "gene_symbol": "WFDC10B"
}